negative regulation of locomotion involved in locomotory behavior [GO:0090327] (biological process) Definition: Any process that decreases the frequency, rate, or extent of the self-propelled movement of a cell or organism from one location to another in a behavioral context; the aspect of locomotory behavior having to do with movement. Relationships: is_a GO:0040013; is a type of GO:0048521; is a type of regulation of locomotion involved in locomotory behavior [GO:0090325]; negatively regulates locomotion involved in locomotory behavior [GO:0031987] Sources: GOC:dph, GOC:kmv, GOC:tb